{
  "gene": "UniProtKB:A5PKW4",
  "term_label": "vesicle-mediated transport",
  "term_id": "GO:0016192",
  "gene_name": "PH and SEC7 domain-containing protein 1",
  "gene_symbol": "PSD"
}